chromaffin granule [GO:0042583] (cellular component) References: PMID:19158310, PMID:1961743 Sources: GOC:jl Relationships: is a type of secretory granule [GO:0030141] Definition: Specialized secretory vesicle found in the cells of adrenal glands and various other organs, which is concerned with the synthesis, storage, metabolism, and secretion of epinephrine and norepinephrine.